{
  "term_id": "GO:0005886",
  "gene": "UniProtKB:Q96LB1",
  "term_label": "plasma membrane",
  "gene_symbol": "MRGPRX2",
  "gene_name": "Mas-related G-protein coupled receptor member X2"
}